{
  "gene": "UniProtKB:Q5JVF3",
  "term_id": "GO:0000973",
  "gene_symbol": "PCID2",
  "gene_name": "PCI domain-containing protein 2",
  "term_label": "post-transcriptional tethering of RNA polymerase II gene DNA at nuclear periphery"
}